{
  "gene_symbol": "MYO1D",
  "term_label": "endocytosis",
  "gene_name": "Unconventional myosin-Id",
  "gene": "UniProtKB:O94832",
  "term_id": "GO:0006897"
}